regulation of mesenchymal to epithelial transition involved in metanephros morphogenesis [GO:0003339] (biological process) Definition: Any process that modulates the rate, frequency or extent of the transition where a mesenchymal cell establishes apical/basolateral polarity,forms intercellular adhesive junctions, synthesizes basement membrane components and becomes an epithelial cell that will contribute to the shaping of the metanephros. Sources: GOC:dph Subtypes: negative regulation of mesenchymal to epithelial transition involved in metanephros morphogenesis [GO:0003340], positive regulation of mesenchymal to epithelial transition involved in metanephros morphogenesis [GO:0072108] Relationships: is a type of regulation of epithelial cell differentiation involved in kidney development [GO:2000696]; regulates mesenchymal to epithelial transition involved in metanephros morphogenesis [GO:0003337]